{
  "gene_name": "ATP-dependent 6-phosphofructokinase, platelet type",
  "term_id": "GO:0070095",
  "gene_symbol": "PFKP",
  "term_label": "fructose-6-phosphate binding",
  "gene": "UniProtKB:Q01813"
}